{
  "term_label": "Unknown molecular function",
  "gene_symbol": "LCA10",
  "gene": "UniProtKB:Q71F78",
  "term_id": "UNKNOWN:0001",
  "gene_name": "Putative lung carcinoma-associated protein 10"
}